{
  "term_label": "mitochondrial transmembrane transport",
  "gene_symbol": "SFXN4",
  "gene": "UniProtKB:Q6P4A7",
  "term_id": "GO:1990542",
  "gene_name": "Sideroflexin-4"
}